{
  "gene_name": "UDP-glucuronosyltransferase 1A3",
  "gene": "UniProtKB:P35503",
  "term_label": "liver development",
  "gene_symbol": "UGT1A3",
  "term_id": "GO:0001889"
}